bombesin receptor activity [GO:0004946] (molecular function) Relationships: is a type of GO:0008188; is part of bombesin receptor signaling pathway [GO:0031989] Sources: GOC:ai Definition: Combining with bombesin to initiate a change in cell activity.